{
  "term_label": "protein kinase binding",
  "gene": "UniProtKB:P31947",
  "gene_name": "14-3-3 protein sigma",
  "term_id": "GO:0019901",
  "gene_symbol": "SFN"
}